chlorophyll catabolic process [GO:0015996] (biological process) Relationships: is a type of porphyrin-containing compound catabolic process [GO:0006787]; is a type of chlorophyll metabolic process [GO:0015994]; is a type of GO:0046149 Also known as: chlorophyll breakdown, chlorophyll catabolism, chlorophyll degradation Regulation: regulated by GO:0010271; negatively regulated by GO:1903647; positively regulated by positive regulation of chlorophyll catabolic process [GO:1903648] Definition: The chemical reactions and pathways resulting in the breakdown of chlorophyll, any compound of magnesium complexed in a porphyrin (tetrapyrrole) ring and which functions as a photosynthetic pigment, into less complex products. Subtypes: bacteriochlorophyll catabolic process [GO:0030495], chlorophyll a catabolic process [GO:0033310] Sources: GOC:jl